{
  "gene_symbol": "OSBPL1A",
  "gene_name": "Oxysterol-binding protein-related protein 1",
  "gene": "UniProtKB:Q9BXW6",
  "term_label": "perinuclear endoplasmic reticulum",
  "term_id": "GO:0097038"
}